{
  "gene_name": "Nuclear receptor subfamily 4 group A member 1",
  "term_id": "GO:0005667",
  "gene_symbol": "NR4A1",
  "gene": "UniProtKB:P22736",
  "term_label": "transcription regulator complex"
}